regulation of cell morphogenesis involved in conjugation with cellular fusion [GO:1905708] (biological process) Definition: Any process that modulates the location, frequency, rate or extent of cell morphogenesis involved in conjugation with cellular fusion. References: PMID:23200991 Sources: GOC:TermGenie, GO_REF:0000058 Also known as: regulation of shmoo orientation, regulation of shmooing Relationships: is a type of regulation of cell morphogenesis [GO:0022604]; regulates cell morphogenesis involved in conjugation with cellular fusion [GO:0000753]